negative regulation of adenylate cyclase activity [GO:0007194] (biological process) Definition: Any process that stops, prevents, or reduces the frequency, rate or extent of adenylate cyclase activity. Also known as: down regulation of adenylate cyclase activity, down-regulation of adenylate cyclase activity, downregulation of adenylate cyclase activity, negative regulation of adenylyl cyclase activity, inhibition of adenylate cyclase activity, adenylate cyclase inhibitor Relationships: is a type of negative regulation of catalytic activity [GO:0043086]; is a type of GO:0045761; negatively regulates adenylate cyclase activity [GO:0004016] Sources: GOC:go_curators